{
  "gene_symbol": "GSTA1",
  "term_label": "cytosol",
  "gene": "UniProtKB:P08263",
  "term_id": "GO:0005829",
  "gene_name": "Glutathione S-transferase A1"
}